{
  "gene": "UniProtKB:O75312",
  "term_label": "axon",
  "gene_symbol": "ZPR1",
  "term_id": "GO:0030424",
  "gene_name": "Zinc finger protein ZPR1"
}